{
  "gene": "UniProtKB:O60674",
  "gene_symbol": "JAK2",
  "gene_name": "Tyrosine-protein kinase JAK2",
  "term_id": "GO:0007259",
  "term_label": "cell surface receptor signaling pathway via JAK-STAT"
}